{
  "gene_name": "Serine_threonine-protein kinase TBK1",
  "term_label": "activation of innate immune response",
  "gene": "UniProtKB:Q9UHD2",
  "gene_symbol": "TBK1",
  "term_id": "GO:0002218"
}